nucleoplasm [GO:0005654] (cellular component) Definition: That part of the nuclear content other than the chromosomes or the nucleolus. Relationships: is a type of cellular anatomical structure [GO:0110165]; is part of GO:0031981 Sources: GOC:ma, ISBN:0124325653